{
  "gene_symbol": "IKBKB",
  "term_label": "tumor necrosis factor-mediated signaling pathway",
  "gene": "UniProtKB:O14920",
  "term_id": "GO:0033209",
  "gene_name": "Inhibitor of nuclear factor kappa-B kinase subunit beta"
}